{
  "gene_name": "SLAIN motif-containing protein 1",
  "term_label": "microtubule plus-end",
  "gene_symbol": "SLAIN1",
  "gene": "UniProtKB:Q8ND83",
  "term_id": "GO:0035371"
}